{
  "term_id": "GO:0097527",
  "gene_symbol": "MLKL",
  "gene": "UniProtKB:Q8NB16",
  "gene_name": "Mixed lineage kinase domain-like protein",
  "term_label": "necroptotic signaling pathway"
}